positive regulation of actin filament bundle assembly [GO:0032233] (biological process) Definition: Any process that activates or increases the frequency, rate or extent of the assembly of actin filament bundles. Also known as: up regulation of actin filament bundle formation, up-regulation of actin filament bundle formation, upregulation of actin filament bundle formation, activation of actin filament bundle formation, stimulation of actin filament bundle formation Subtypes: GO:0051496, GO:0090338 Sources: GOC:mah Relationships: is a type of GO:0032231; is a type of positive regulation of cellular component biogenesis [GO:0044089]; is a type of positive regulation of cytoskeleton organization [GO:0051495]; is a type of positive regulation of supramolecular fiber organization [GO:1902905]; positively regulates GO:0051017